{
  "gene": "UniProtKB:Q99848",
  "gene_name": "Probable rRNA-processing protein EBP2",
  "gene_symbol": "EBNA1BP2",
  "term_label": "nuclear periphery",
  "term_id": "GO:0034399"
}